{
  "term_id": "GO:0061928",
  "gene_symbol": "CHAC1",
  "term_label": "glutathione specific gamma-glutamylcyclotransferase activity",
  "gene_name": "Glutathione-specific gamma-glutamylcyclotransferase 1",
  "gene": "UniProtKB:Q9BUX1"
}